appressorium formation [GO:0075016] (biological process) Regulation: regulated by regulation of appressorium formation [GO:0075017]; positively regulated by GO:0075018; negatively regulated by negative regulation of appressorium formation [GO:0075019] Relationships: is a type of formation of infection structure [GO:0075015] Definition: The process in which a swollen, flattened portion of a symbiont filament is formed on or near its host organism, to adhere to and for the purpose of penetrating the host surface. Also known as: appressorium formation for entry into host, on or near host, formation of an appressorium by symbiont on or near host, appressorium formation on or near host Sources: GOC:pamgo_curators